{
  "gene_name": "Elongation of very long chain fatty acids protein 5",
  "gene": "UniProtKB:Q9NYP7",
  "gene_symbol": "ELOVL5",
  "term_label": "fatty acid elongation, polyunsaturated fatty acid",
  "term_id": "GO:0034626"
}